{
  "gene": "UniProtKB:Q14654",
  "term_id": "GO:0005886",
  "gene_name": "ATP-sensitive inward rectifier potassium channel 11",
  "gene_symbol": "KCNJ11",
  "term_label": "plasma membrane"
}